regulation of cellular response to macrophage colony-stimulating factor stimulus [GO:1903972] (biological process) Definition: Any process that modulates the frequency, rate or extent of cellular response to macrophage colony-stimulating factor stimulus. References: PMID:19100238 Sources: GOC:BHF, GOC:TermGenie, GOC:nc, GO_REF:0000058 Also known as: regulation of cellular response to M-CSF stimulus, regulation of cellular response to macrophage colony-stimulating factor Relationships: is a type of regulation of response to macrophage colony-stimulating factor [GO:1903969]; regulates cellular response to macrophage colony-stimulating factor stimulus [GO:0036006] Subtypes: regulation of macrophage colony-stimulating factor signaling pathway [GO:1902226], negative regulation of cellular response to macrophage colony-stimulating factor stimulus [GO:1903973], GO:1903974